regulation of atrichoblast fate specification [GO:0010058] (biological process) Definition: Any process that modulates atrichoblast fate specification. Sources: GOC:tb Relationships: is_a regulation of cell fate specification [GO:0042659]; is a type of GO:1903888; regulates atrichoblast fate specification [GO:0010056] Subtypes: positive regulation of atrichoblast fate specification [GO:0010059], negative regulation of atrichoblast fate specification [GO:0010060]